{
  "gene": "UniProtKB:O76064",
  "term_id": "GO:0006302",
  "term_label": "double-strand break repair",
  "gene_symbol": "RNF8",
  "gene_name": "E3 ubiquitin-protein ligase RNF8"
}